{
  "gene": "UniProtKB:Q6QHC5",
  "term_label": "Unknown cellular component",
  "gene_symbol": "DEGS2",
  "gene_name": "Sphingolipid delta(4)-desaturase_C4-monooxygenase DES2",
  "term_id": "UNKNOWN:0003"
}